branched-chain-2-oxoacid decarboxylase activity [GO:0047433] (molecular function) Sources: EC:4.1.1.72, RHEA:21108 Also known as: (3S)-3-methyl-2-oxopentanoate carboxy-lyase (2-methylbutanal-forming), (3S)-3-methyl-2-oxopentanoate carboxy-lyase activity, BCKA, branched-chain alpha-keto acid decarboxylase activity, branched-chain keto acid decarboxylase activity, branched-chain oxo acid decarboxylase activity Definition: Catalysis of the reaction: (S)-3-methyl-2-oxopentanoate + H+ = 2-methylbutanal + CO2. Relationships: is a type of carboxy-lyase activity [GO:0016831]